closure of embryonic heart tube [GO:0003153] (biological process) Sources: GOC:mtg_heart Definition: Creation of the central hole of the embryonic heart tube by sealing the edges of an epithelial fold. Relationships: is a type of GO:0060606; is part of embryonic heart tube formation via epithelial folding [GO:0003145]